histamine transmembrane transporter activity [GO:0160173] (molecular function) Relationships: is a type of azole transmembrane transporter activity [GO:1901474] Definition: Enables the transfer of histamine from one side of a membrane to the other. References: PMID:36288320 Subtypes: L-histidine:histamine antiporter activity [GO:0070907]